{
  "gene": "UniProtKB:Q9NP91",
  "term_label": "proline:sodium symporter activity",
  "gene_name": "Sodium- and chloride-dependent transporter XTRP3",
  "gene_symbol": "SLC6A20",
  "term_id": "GO:0005298"
}